2'-deoxyribonucleotide metabolic process [GO:0009394] (biological process) Definition: The chemical reactions and pathways involving a 2'-deoxyribonucleotide, a compound consisting of 2'-deoxyribonucleoside (a base linked to a 2'-deoxyribose sugar) esterified with a phosphate group at either the 3' or 5'-hydroxyl group of the sugar. Subtypes: purine deoxyribonucleotide metabolic process [GO:0009151], pyrimidine deoxyribonucleotide metabolic process [GO:0009219], 2'-deoxyribonucleotide biosynthetic process [GO:0009265] Also known as: 2'-deoxyribonucleotide metabolism Sources: GOC:mah Relationships: is a type of deoxyribonucleotide metabolic process [GO:0009262]